{
  "term_id": "GO:0005739",
  "gene": "UniProtKB:P05177",
  "gene_symbol": "CYP1A2",
  "gene_name": "Cytochrome P450 1A2",
  "term_label": "mitochondrion"
}